{
  "term_label": "C-C chemokine receptor activity",
  "gene_name": "Atypical chemokine receptor 3",
  "term_id": "GO:0016493",
  "gene": "UniProtKB:P25106",
  "gene_symbol": "ACKR3"
}